{
  "term_id": "GO:0005886",
  "term_label": "plasma membrane",
  "gene": "UniProtKB:Q8NCM2",
  "gene_symbol": "KCNH5",
  "gene_name": "Potassium voltage-gated channel subfamily H member 5"
}